7-methylthiopropyl glucosinolate S-oxygenase activity [GO:0080106] (molecular function) Definition: Catalysis of the reaction: 7-methylthiopropyl-glucosinolate = 7-methylsulfinylpropyl-glucosinolate. References: PMID:18799661 Relationships: is a type of oxidoreductase activity, acting on paired donors, with incorporation or reduction of molecular oxygen [GO:0016705]